{
  "gene_name": "Tumor necrosis factor receptor superfamily member 10B",
  "term_label": "Unknown molecular function",
  "gene": "UniProtKB:O14763",
  "gene_symbol": "TNFRSF10B",
  "term_id": "UNKNOWN:0001"
}